imaginal disc lineage restriction [GO:0035161] (biological process) References: PMID:10625531, PMID:9374402 Sources: GOC:bf Subtypes: dorsal/ventral lineage restriction, imaginal disc [GO:0007451], GO:0048099 Definition: Formation and/or maintenance of a lineage boundary between compartments in an imaginal disc that cells cannot cross, thus separating the populations of cells in each compartment. Relationships: is a type of pattern specification process [GO:0007389]; is part of imaginal disc pattern formation [GO:0007447]